{
  "gene": "UniProtKB:P30838",
  "term_label": "aldehyde dehydrogenase (NAD+) activity",
  "term_id": "GO:0004029",
  "gene_name": "Aldehyde dehydrogenase, dimeric NADP-preferring",
  "gene_symbol": "ALDH3A1"
}